{
  "term_id": "UNKNOWN:0001",
  "gene_name": "T cell receptor gamma variable 8",
  "term_label": "Unknown molecular function",
  "gene_symbol": "TRGV8",
  "gene": "UniProtKB:A0A0C4DH27"
}